{
  "term_label": "Unknown molecular function",
  "gene": "UniProtKB:P15421",
  "term_id": "UNKNOWN:0001",
  "gene_name": "Glycophorin-E",
  "gene_symbol": "GYPE"
}